box C/D methylation guide snoRNP complex binding [GO:0062064] (molecular function) Definition: Binding to a box C/D methylation guide snoRNP complex. Relationships: is a type of snoRNP binding [GO:0030519] References: PMID:10679015